{
  "term_label": "microtubule-based process",
  "gene": "UniProtKB:Q9BVG8",
  "gene_symbol": "KIFC3",
  "term_id": "GO:0007017",
  "gene_name": "Kinesin-like protein KIFC3"
}